{
  "gene": "UniProtKB:Q9H0R6",
  "term_label": "glutaminyl-tRNAGln biosynthesis via transamidation",
  "term_id": "GO:0070681",
  "gene_name": "Glutamyl-tRNA(Gln) amidotransferase subunit A, mitochondrial",
  "gene_symbol": "QRSL1"
}